{
  "term_label": "oxidoreductase activity, acting on paired donors, with incorporation or reduction of molecular oxygen, reduced flavin or flavoprotein as one donor, and incorporation of one atom of oxygen",
  "term_id": "GO:0016712",
  "gene_name": "Cytochrome P450 2C9",
  "gene_symbol": "CYP2C9",
  "gene": "UniProtKB:P11712"
}